{
  "gene": "UniProtKB:P13569",
  "gene_symbol": "CFTR",
  "term_label": "ABC-type transporter activity",
  "gene_name": "Cystic fibrosis transmembrane conductance regulator",
  "term_id": "GO:0140359"
}